{
  "gene": "UniProtKB:A6ND91",
  "gene_name": "Aspartate dehydrogenase domain-containing protein",
  "term_label": "Unknown cellular component",
  "gene_symbol": "ASPDH",
  "term_id": "UNKNOWN:0003"
}